adaptive immune memory response involving T cells and B cells [GO:0090717] (biological process) Relationships: is_a adaptive immune response based on somatic recombination of immune receptors built from immunoglobulin superfamily domains [GO:0002460]; is a type of adaptive immune memory response [GO:0090716] References: PMID:26831526 Sources: GOC:add Definition: An immune response mediated by reactivated memory T cells and B cells and directed against a previously encountered antigen, being quicker and quantitatively better compared with the primary response.